{
  "term_id": "GO:0047631",
  "gene": "UniProtKB:Q9UKK9",
  "gene_symbol": "NUDT5",
  "term_label": "ADP-ribose diphosphatase activity",
  "gene_name": "ADP-sugar pyrophosphatase"
}